horizontal gene transfer [GO:0009292] (biological process) Subtypes: unidirectional conjugation [GO:0009291], transduction [GO:0009293], DNA-mediated transformation [GO:0009294] Relationships: is a type of cellular process [GO:0009987] References: PMID:26184597 Definition: The introduction of genetic information into a cell to create a genetically different individual, without production of new individuals. Also known as: genetic exchange, genetic transfer, lateral gene transfer